{
  "gene_name": "AF4_FMR2 family member 3",
  "gene": "UniProtKB:P51826",
  "term_id": "GO:0006354",
  "gene_symbol": "AFF3",
  "term_label": "DNA-templated transcription elongation"
}